{
  "term_label": "anatomical structure morphogenesis",
  "gene_name": "Hepatocyte nuclear factor 3-alpha",
  "term_id": "GO:0009653",
  "gene": "UniProtKB:P55317",
  "gene_symbol": "FOXA1"
}